phloem transport [GO:0010233] (BP) Subtypes: phloem loading [GO:0110126], phloem unloading [GO:0110127], xylem-to-phloem iron transport [GO:1990388] Definition: The directed movement of substances, into, out of or within the phloem during long distance transport between source and sink tissues. References: PMID:19025382 Sources: GOC:sm Relationships: is a type of vascular transport [GO:0010232]